{
  "gene_symbol": "FSCN1",
  "gene": "UniProtKB:Q16658",
  "gene_name": "Fascin",
  "term_id": "GO:0007163",
  "term_label": "establishment or maintenance of cell polarity"
}